diacylglycerol-sterol O-acyltransferase activity [GO:0047195] (molecular function) Sources: EC:2.3.1.73, MetaCyc:2.3.1.73-RXN Relationships: is a type of O-acyltransferase activity [GO:0008374] Definition: Catalysis of the reaction: sterol + 1,2-diacylglycerol = sterol ester + acylglycerol. Also known as: 1,2-diacyl-sn-glycerol:sterol O-acyltransferase activity, 1,2-diacyl-sn-glycerol:sterol acyl transferase activity